{
  "term_label": "cytoplasm",
  "gene_name": "Putative ADP-ribosylation factor-like protein 5C",
  "gene_symbol": "ARL5C",
  "term_id": "GO:0005737",
  "gene": "UniProtKB:A6NH57"
}